P5 peroxisome [GO:0019823] (cellular component) Definition: A subform of peroxisome that corresponds to an intermediate in a peroxisome assembly pathway, which operates by conversion of peroxisomal subforms in the direction P1, P2 -> P3 -> P4 -> P5 -> P6. P5 peroxisomes are distinguished from the other subforms on the bases of buoyant density and protein content. Note: Note that this peroxisome assembly pathway is described in the yeast Yarrowia lipolytica. See also the cellular component terms 'P1 peroxisome ; GO:0019819', 'P2 peroxisome ; GO:0019820', 'P3 peroxisome ; GO:0019821', 'P4 peroxisome ; GO:0019822', and 'P6 peroxisome ; GO:0019824'. Also known as: peroxisome vesicle Relationships: is a type of peroxisome [GO:0005777] References: PMID:10629216